{
  "gene_symbol": "GP6",
  "term_label": "immune receptor activity",
  "gene": "UniProtKB:Q9HCN6",
  "term_id": "GO:0140375",
  "gene_name": "Platelet glycoprotein VI"
}